B875 antenna complex [GO:0030080] (cellular component) Relationships: is_a GO:0032991; is part of GO:0030078 Sources: GOC:kd Also known as: LH1 complex, light harvesting complex I Definition: Protein complex that surrounds and transfers excitation energy directly to the bacterial reaction center; binds bacteriochlorophyll a and has a single absorption band between 870 and 890 nm.